{
  "term_id": "GO:0006357",
  "gene_symbol": "FOXO3",
  "gene": "UniProtKB:O43524",
  "gene_name": "Forkhead box protein O3",
  "term_label": "regulation of transcription by RNA polymerase II"
}